{
  "term_id": "GO:0003712",
  "gene": "UniProtKB:P98168",
  "gene_name": "Zinc finger X-linked protein ZXDA",
  "gene_symbol": "ZXDA",
  "term_label": "transcription coregulator activity"
}